{
  "term_id": "UNKNOWN:0001",
  "gene": "UniProtKB:Q5VSR9",
  "gene_symbol": "SPANXN1",
  "term_label": "Unknown molecular function",
  "gene_name": "Sperm protein associated with the nucleus on the X chromosome N1"
}